peroxisome fission [GO:0016559] (biological process) References: PMID:11687502, PMID:14754507 Sources: GOC:mah Definition: The division of a mature peroxisome within a cell to form two or more separate peroxisome compartments. Relationships: is a type of GO:0048285; is part of peroxisome organization [GO:0007031] Also known as: peroxisome division, peroxisome proliferation